{
  "term_id": "GO:0005634",
  "gene": "UniProtKB:Q96NY9",
  "gene_name": "Crossover junction endonuclease MUS81",
  "gene_symbol": "MUS81",
  "term_label": "nucleus"
}